histone methyltransferase binding [GO:1990226] (molecular function) References: PMID:19486527 Sources: GOC:BHF, GOC:ame Relationships: is a type of enzyme binding [GO:0019899] Definition: Binding to a histone methyltransferase enzyme.